{
  "gene": "UniProtKB:O94900",
  "term_id": "GO:0006357",
  "gene_symbol": "TOX",
  "gene_name": "Thymocyte selection-associated high mobility group box protein TOX",
  "term_label": "regulation of transcription by RNA polymerase II"
}